{
  "term_id": "GO:0006541",
  "gene": "UniProtKB:Q9NQR4",
  "term_label": "glutamine metabolic process",
  "gene_symbol": "NIT2",
  "gene_name": "Omega-amidase NIT2"
}